{
  "term_id": "GO:0005783",
  "gene": "UniProtKB:Q8IVT5",
  "term_label": "endoplasmic reticulum",
  "gene_symbol": "KSR1",
  "gene_name": "Kinase suppressor of Ras 1"
}